{
  "gene_symbol": "WTIP",
  "gene": "UniProtKB:A6NIX2",
  "term_id": "GO:0001666",
  "term_label": "response to hypoxia",
  "gene_name": "Wilms tumor protein 1-interacting protein"
}